{
  "gene": "UniProtKB:P26038",
  "term_label": "plasma membrane",
  "term_id": "GO:0005886",
  "gene_symbol": "MSN",
  "gene_name": "Moesin"
}